{
  "term_label": "metal ion binding",
  "gene": "UniProtKB:P61604",
  "term_id": "GO:0046872",
  "gene_symbol": "HSPE1",
  "gene_name": "10 kDa heat shock protein, mitochondrial"
}